{
  "term_label": "protein localization to plasma membrane",
  "term_id": "GO:0072659",
  "gene_symbol": "EFR3B",
  "gene": "UniProtKB:Q9Y2G0",
  "gene_name": "Protein EFR3 homolog B"
}